{
  "gene": "UniProtKB:Q8N5J2",
  "gene_symbol": "MINDY1",
  "term_id": "GO:0005654",
  "gene_name": "Ubiquitin carboxyl-terminal hydrolase MINDY-1",
  "term_label": "nucleoplasm"
}